mesonephric capsule morphogenesis [GO:0061286] (biological process) Sources: GOC:mtg_kidney_jan10 Definition: The process in which the anatomical structures of the mesonephric capsule are generated and organized. The mesonephric capsule is the tough fibrous layer surrounding the mesonephros, covered in a thick layer of perinephric adipose tissue. It provides some protection from trauma and damage. Relationships: is_a renal capsule morphogenesis [GO:0072128]; is part of mesonephric capsule development [GO:0061285]